{
  "gene_symbol": "FAM47A",
  "term_id": "UNKNOWN:0002",
  "term_label": "Unknown biological process",
  "gene": "UniProtKB:Q5JRC9",
  "gene_name": "Protein FAM47A"
}